{
  "gene_symbol": "CCL28",
  "gene_name": "C-C motif chemokine 28",
  "gene": "UniProtKB:Q9NRJ3",
  "term_id": "GO:0006954",
  "term_label": "inflammatory response"
}